{
  "gene_symbol": "SDHC",
  "term_id": "GO:0045273",
  "gene": "UniProtKB:Q99643",
  "term_label": "respiratory chain complex II (succinate dehydrogenase)",
  "gene_name": "Succinate dehydrogenase cytochrome b560 subunit, mitochondrial"
}